lead sulfide oxidation [GO:0019327] (biological process) Relationships: is a type of energy derivation by oxidation of reduced inorganic compounds [GO:0015975] Also known as: lead sulphide oxidation, oxidation of galena, oxidation of lead sulfide Definition: The chemical reactions and pathways resulting in the conversion of lead sulfide to lead sulfate. Sources: MetaCyc:P301-PWY